{
  "term_label": "cytoplasm",
  "gene_name": "Tubulinyl-Tyr carboxypeptidase 2",
  "term_id": "GO:0005737",
  "gene_symbol": "VASH2",
  "gene": "UniProtKB:Q86V25"
}